{
  "gene": "UniProtKB:Q9BXU1",
  "gene_symbol": "STK31",
  "term_id": "GO:0004521",
  "gene_name": "Serine_threonine-protein kinase 31",
  "term_label": "RNA endonuclease activity"
}